regulation of NK T cell activation [GO:0051133] (biological process) Definition: Any process that modulates the frequency, rate or extent of natural killer T cell activation. References: PMID:12154375, PMID:9133426 Sources: ISBN:0781735149 Also known as: regulation of NK T lymphocyte activation, regulation of NK T-cell activation, regulation of NK T-lymphocyte activation, regulation of NKT cell activation, regulation of NT cell activation, regulation of natural T cell activation, regulation of natural killer T cell activation Relationships: is a type of regulation of alpha-beta T cell activation [GO:0046634]; regulates NK T cell activation [GO:0051132] Subtypes: negative regulation of NK T cell activation [GO:0051134], positive regulation of NK T cell activation [GO:0051135], regulation of NK T cell proliferation [GO:0051140]